{
  "gene_symbol": "HSP90AA1",
  "term_label": "ATP hydrolysis activity",
  "gene_name": "Heat shock protein HSP 90-alpha",
  "term_id": "GO:0016887",
  "gene": "UniProtKB:P07900"
}